{
  "term_id": "GO:0000981",
  "gene_symbol": "MYB",
  "gene_name": "Transcriptional activator Myb",
  "gene": "UniProtKB:P10242",
  "term_label": "DNA-binding transcription factor activity, RNA polymerase II-specific"
}